{
  "gene_symbol": "PTPN18",
  "gene_name": "Tyrosine-protein phosphatase non-receptor type 18",
  "term_id": "GO:0005737",
  "gene": "UniProtKB:Q99952",
  "term_label": "cytoplasm"
}